{
  "gene_name": "Outer dense fiber protein 3-like protein 1",
  "gene_symbol": "CIMAP1C",
  "term_label": "cytoskeleton",
  "term_id": "GO:0005856",
  "gene": "UniProtKB:Q8IXM7"
}